{
  "gene_symbol": "LINC00336",
  "term_id": "UNKNOWN:0002",
  "gene_name": "Putative uncharacterized protein encoded by LINC00336",
  "gene": "UniProtKB:Q6ZUF6",
  "term_label": "Unknown biological process"
}